{
  "term_label": "microtubule",
  "gene": "UniProtKB:Q12840",
  "gene_symbol": "KIF5A",
  "gene_name": "Kinesin heavy chain isoform 5A",
  "term_id": "GO:0005874"
}